protein carbamoylation [GO:0046944] (biological process) Also known as: protein amino acid carbamoylation Sources: GOC:ai Relationships: is a type of protein modification process [GO:0036211] Definition: The addition of a carbamoyl group to a protein amino acid. A carbamoyl group is the acyl group -CO-NH2.